{
  "term_id": "GO:0007519",
  "gene_symbol": "RTL1",
  "gene_name": "Retrotransposon-like protein 1",
  "gene": "UniProtKB:A6NKG5",
  "term_label": "skeletal muscle tissue development"
}